deaminated base DNA N-glycosylase activity [GO:0097506] (molecular function) Relationships: is a type of DNA N-glycosylase activity [GO:0019104] Also known as: DNA glycosylase activity acting on deaminated bases, deaminated base DNA glycosylase activity References: PMID:18789404 Sources: GOC:al Definition: DNA N-glycosylase activity acting on deaminated bases. Subtypes: uracil DNA N-glycosylase activity [GO:0004844], hypoxanthine DNA N-glycosylase activity [GO:0097507], xanthine DNA N-glycosylase activity [GO:0097508], oxanine DNA N-glycosylase activity [GO:0097509]